{
  "gene": "UniProtKB:Q5SV17",
  "term_id": "UNKNOWN:0002",
  "gene_symbol": "TMEM240",
  "gene_name": "Transmembrane protein 240",
  "term_label": "Unknown biological process"
}